{
  "term_label": "long-chain fatty acid biosynthetic process",
  "gene_symbol": "ASAH2",
  "gene": "UniProtKB:Q9NR71",
  "term_id": "GO:0042759",
  "gene_name": "Neutral ceramidase"
}